eukaryotic translation initiation factor 2B complex assembly [GO:1905173] (BP) Also known as: eIF-2B assembly, eIF-2B formation, eif2B assembly, eif2B formation, eukaryotic translation initiation factor 2B complex formation Relationships: is a type of protein-containing complex assembly [GO:0065003] Definition: The aggregation, arrangement and bonding together of a set of components to form an eukaryotic translation initiation factor 2B complex. References: PMID:27023709 Sources: GOC:TermGenie, GO_REF:0000079